{
  "gene": "UniProtKB:Q9BWW7",
  "term_label": "Unknown cellular component",
  "gene_symbol": "SCRT1",
  "term_id": "UNKNOWN:0003",
  "gene_name": "Transcriptional repressor scratch 1"
}